thermosensory behavior [GO:0040040] (biological process) Relationships: is a type of behavior [GO:0007610]; is a type of response to temperature stimulus [GO:0009266] Definition: Behavior that is dependent upon the sensation of temperature. Also known as: behavioral response to temperature stimulus, behavioural response to temperature stimulus, thermosensory behaviour Sources: GOC:ems